{
  "gene": "UniProtKB:P51178",
  "gene_name": "1-phosphatidylinositol 4,5-bisphosphate phosphodiesterase delta-1",
  "term_label": "cytoplasm",
  "term_id": "GO:0005737",
  "gene_symbol": "PLCD1"
}